BRCA1-A complex [GO:0070531] (CC) Definition: A protein complex that contains the BRCA1-BARD1 heterodimer, RAP80/UIMC1, BRCC3/BRCC36, BRE/BRCC45, FAM175A/CCDC98/Abraxas and MERIT40/NBA1, and specifically recognizes and binds K63-linked polyubiquitin chains present on histone H2A and H2AX at DNA damage sites. References: PMID:19261749 Sources: GOC:mah Relationships: is a type of GO:0140513